{
  "gene_name": "Carcinoembryonic antigen-related cell adhesion molecule 4",
  "gene_symbol": "CEACAM4",
  "term_label": "regulation of immune system process",
  "term_id": "GO:0002682",
  "gene": "UniProtKB:O75871"
}